{
  "gene_symbol": "IZUMO4",
  "term_label": "Unknown cellular component",
  "term_id": "UNKNOWN:0003",
  "gene_name": "Izumo sperm-egg fusion protein 4",
  "gene": "UniProtKB:Q1ZYL8"
}